{
  "gene_name": "Protocadherin beta-10",
  "term_label": "cell adhesion",
  "gene_symbol": "PCDHB10",
  "term_id": "GO:0007155",
  "gene": "UniProtKB:Q9UN67"
}